{
  "gene_symbol": "DEFB129",
  "term_label": "Unknown biological process",
  "term_id": "UNKNOWN:0002",
  "gene_name": "Beta-defensin 129",
  "gene": "UniProtKB:Q9H1M3"
}